{
  "term_id": "GO:0090280",
  "term_label": "positive regulation of calcium ion import",
  "gene_name": "Galectin-3",
  "gene_symbol": "LGALS3",
  "gene": "UniProtKB:P17931"
}